{
  "gene_symbol": "RCAN1",
  "term_label": "cytoplasm",
  "gene": "UniProtKB:P53805",
  "term_id": "GO:0005737",
  "gene_name": "Calcipressin-1"
}